{
  "term_id": "GO:0005886",
  "gene": "UniProtKB:O76100",
  "term_label": "plasma membrane",
  "gene_symbol": "OR7A10",
  "gene_name": "Olfactory receptor 7A10"
}